toll-like receptor 6 signaling pathway [GO:0034150] (BP) Also known as: TLR6 signaling pathway, toll-like receptor 6 signalling pathway References: PMID:16551253, PMID:17328678 Sources: GOC:add Definition: The series of molecular signals initiated by a ligand binding to toll-like receptor 6. Regulation: regulated by GO:0034151; negatively regulated by negative regulation of toll-like receptor 6 signaling pathway [GO:0034152]; positively regulated by GO:0034153 Relationships: is a type of GO:0140895